{
  "gene": "UniProtKB:Q8TBE1",
  "term_label": "signaling receptor binding",
  "term_id": "GO:0005102",
  "gene_symbol": "CNIH3",
  "gene_name": "Protein cornichon homolog 3"
}